epicardium-derived cardiac vascular smooth muscle cell differentiation [GO:0060983] (biological process) Sources: GOC:mtg_heart Definition: The process in which a relatively unspecialized cell derived from the epicardium acquires specialized features of a cardiac vascular smooth muscle cell. A cardiac vascular smooth muscle cell covers the heart vasculature and lacks transverse striations in its constituent fibers. Relationships: is_a GO:0060947